{
  "gene": "UniProtKB:Q8WYK2",
  "term_id": "GO:0000981",
  "term_label": "DNA-binding transcription factor activity, RNA polymerase II-specific",
  "gene_symbol": "JDP2",
  "gene_name": "Jun dimerization protein 2"
}